{
  "gene_name": "Zinc finger protein 454",
  "term_label": "RNA polymerase II cis-regulatory region sequence-specific DNA binding",
  "gene": "UniProtKB:Q8N9F8",
  "term_id": "GO:0000978",
  "gene_symbol": "ZNF454"
}